{
  "term_label": "septin ring",
  "gene_symbol": "SEPTIN1",
  "gene": "UniProtKB:Q8WYJ6",
  "gene_name": "Septin-1",
  "term_id": "GO:0005940"
}